L-ascorbic acid binding [GO:0031418] (molecular function) Definition: Binding to L-ascorbic acid, (2R)-2-[(1S)-1,2-dihydroxyethyl]-4-hydroxy-5-oxo-2,5-dihydrofuran-3-olate; L-ascorbic acid is vitamin C and has co-factor and anti-oxidant activities in many species. Also known as: L-ascorbate binding, vitamin C binding Relationships: is a type of vitamin binding [GO:0019842]; is a type of carboxylic acid binding [GO:0031406]; is a type of GO:0048029; is a type of heterocyclic compound binding [GO:1901363] Sources: GOC:mah